bile acid-gated sodium channel activity [GO:0160228] (molecular function) Definition: Enables the transmembrane transfer of a sodium ion by a channel that opens when bile acid has been bound by the channel complex or one of its constituent parts. Relationships: is a type of GO:0005272 References: PMID:22735174